{
  "gene": "UniProtKB:Q8NEP3",
  "gene_symbol": "DNAAF1",
  "gene_name": "Dynein axonemal assembly factor 1",
  "term_label": "axoneme",
  "term_id": "GO:0005930"
}